{
  "gene_name": "Endoplasmic reticulum membrane adapter protein XK",
  "gene": "UniProtKB:P51811",
  "term_id": "GO:0005789",
  "term_label": "endoplasmic reticulum membrane",
  "gene_symbol": "XK"
}